mitochondrial processing peptidase complex [GO:0017087] (cellular component) Relationships: is a type of mitochondrial protein-containing complex [GO:0098798]; is a type of endopeptidase complex [GO:1905369]; is part of mitochondrial matrix [GO:0005759] Definition: A protein complex consisting of a regulatory subunit (alpha-MPP) and a catalytic subunit (beta-MPP) that catalyzes the release of N-terminal targeting peptides from precursor proteins imported into the mitochondrion. Note: Note that monomeric mitochondrial processing peptidases have been observed. Sources: GOC:mah